replication fork reversal [GO:0071932] (biological process) Relationships: is a type of replication fork processing [GO:0031297] Definition: Replication fork processing that involves the unwinding of blocked forks to form four-stranded structures resembling Holliday junctions, which are subsequently resolved. References: PMID:19406929